{
  "term_id": "GO:0030071",
  "gene_symbol": "MAP3K20",
  "gene_name": "Mitogen-activated protein kinase kinase kinase 20",
  "term_label": "regulation of mitotic metaphase/anaphase transition",
  "gene": "UniProtKB:Q9NYL2"
}